{
  "gene_symbol": "ZNF211",
  "term_label": "nucleus",
  "gene_name": "Zinc finger protein 211",
  "term_id": "GO:0005634",
  "gene": "UniProtKB:Q13398"
}